{
  "gene": "UniProtKB:Q9BXX3",
  "gene_name": "Ankyrin repeat domain-containing protein 30A",
  "term_label": "Unknown cellular component",
  "gene_symbol": "ANKRD30A",
  "term_id": "UNKNOWN:0003"
}